{
  "gene_symbol": "SERPINB12",
  "term_id": "GO:0004867",
  "gene": "UniProtKB:Q96P63",
  "term_label": "serine-type endopeptidase inhibitor activity",
  "gene_name": "Serpin B12"
}